{
  "gene_name": "Uncharacterized protein C22orf31",
  "term_id": "UNKNOWN:0003",
  "term_label": "Unknown cellular component",
  "gene": "UniProtKB:O95567",
  "gene_symbol": "C22orf31"
}